{
  "gene_name": "Tyrosine-protein kinase JAK2",
  "term_label": "erythrocyte differentiation",
  "term_id": "GO:0030218",
  "gene_symbol": "JAK2",
  "gene": "UniProtKB:O60674"
}